ATPase-coupled 2-aminoethylphosphonate transporter activity [GO:0033225] (molecular function) Definition: Enables the directed movement of 2-aminoethylphosphonate from one side of a membrane to the other by catalysis of the reaction: ATP + H2O + 2-aminoethylphosphonate(out) = ADP + phosphate + 2-aminoethylphosphonate(in). Relationships: is a type of ATPase-coupled transmembrane transporter activity [GO:0042626] Also known as: 2-aminoethylphosphonate-transporting ATPase activity, 2-phosphonoethylamine transporting ATPase activity, ATP-dependent 2-aminoethylphosphonate transporter activity, ciliatine transportingATPase activity, 2-aminoethylphosphonate transmembrane transporter activity, 2-aminoethylphosphonate transporting ATPase activity, 2-phosphonoethylamine transmembrane transporter activity, ciliatine transporter activity Note: There is no annotated example of this MF; therefore we cannot classify it more precisely. Sources: GOC:mlg